{
  "gene_symbol": "OTULIN",
  "term_label": "regulation of tumor necrosis factor-mediated signaling pathway",
  "term_id": "GO:0010803",
  "gene_name": "Ubiquitin thioesterase otulin",
  "gene": "UniProtKB:Q96BN8"
}